{
  "term_label": "Unknown cellular component",
  "gene": "UniProtKB:Q5T447",
  "gene_name": "E3 ubiquitin-protein ligase HECTD3",
  "term_id": "UNKNOWN:0003",
  "gene_symbol": "HECTD3"
}